{
  "gene_symbol": "MORC3",
  "term_label": "nucleus",
  "gene": "UniProtKB:Q14149",
  "term_id": "GO:0005634",
  "gene_name": "MORC family CW-type zinc finger protein 3"
}